{
  "gene_symbol": "RARRES2",
  "term_label": "signaling receptor binding",
  "gene": "UniProtKB:Q99969",
  "gene_name": "Retinoic acid receptor responder protein 2",
  "term_id": "GO:0005102"
}